DNA recombinase complex [GO:0097519] (cellular component) Definition: A protein-DNA complex consisting of a higher-order oligomer of strand exchange proteins (recombinases) on single-stranded DNA. References: PMID:10357855 Sources: GOC:cjm Relationships: is a type of GO:0032993